positive regulation of SNARE complex disassembly [GO:0035540] (biological process) Relationships: is a type of regulation of SNARE complex disassembly [GO:0035495]; is a type of positive regulation of protein-containing complex disassembly [GO:0043243]; is a type of positive regulation of transport [GO:0051050]; positively regulates GO:0035494 Definition: Any process that increases the frequency, rate or extent of disassembly of the SNARE complex. The SNARE complex is a protein complex involved in membrane fusion; a stable ternary complex consisting of a four-helix bundle, usually formed from one R-SNARE and three Q-SNAREs with an ionic layer sandwiched between hydrophobic layers. Sources: GOC:rb